regulation of extracellular matrix assembly [GO:1901201] (biological process) Subtypes: negative regulation of extracellular matrix assembly [GO:1901202], positive regulation of extracellular matrix assembly [GO:1901203], GO:1904259 Definition: Any process that modulates the frequency, rate or extent of extracellular matrix assembly. Relationships: is a type of regulation of cellular component biogenesis [GO:0044087]; is a type of regulation of extracellular matrix organization [GO:1903053]; regulates extracellular matrix assembly [GO:0085029] Sources: GOC:BHF, GOC:TermGenie